{
  "gene_name": "RAB11-binding protein RELCH",
  "term_id": "GO:0005802",
  "gene_symbol": "RELCH",
  "term_label": "trans-Golgi network",
  "gene": "UniProtKB:Q9P260"
}